aerial mycelium formation [GO:0097736] (biological process) References: PMID:12832397 Sources: GOC:di Relationships: is a type of anatomical structure development [GO:0048856]; is part of asexual reproduction [GO:0019954] Also known as: aerial hyphal growth, fertile mycelium formation Definition: The process by which hyphae grow in an upward or outward direction from the surface of the substrate; from there, propagative spores develop in or on characteristic structures that are distinctive of some fungal and bacterial species. The species that form an aerial mycelium develop conidiophores at the ends of the aerial hyphae.